{
  "gene_symbol": "ZFY",
  "term_id": "GO:0005634",
  "gene": "UniProtKB:P08048",
  "term_label": "nucleus",
  "gene_name": "Zinc finger Y-chromosomal protein"
}